{
  "term_id": "GO:0004984",
  "gene": "UniProtKB:Q8NGM8",
  "term_label": "olfactory receptor activity",
  "gene_name": "Olfactory receptor 6M1",
  "gene_symbol": "OR6M1"
}